endo-alpha-(2,8)-sialidase activity [GO:0016996] (molecular function) Sources: EC:3.2.1.129 Also known as: alpha-2,8-sialosylhydrolase activity, endo-N-acetylneuraminidase activity, endo-N-acylneuraminidase activity, endoneuraminidase activity, endosialidase activity, poly(alpha-2,8-sialoside) alpha-2,8-sialosylhydrolase activity, poly(alpha-2,8-sialosyl) endo-N-acetylneuraminidase activity, polysialoside (2->8)-alpha-sialosylhydrolase activity Relationships: is a type of GO:0016997 Definition: Catalysis of the endohydrolysis of (2->8)-alpha-sialosyl linkages in oligo- or poly(sialic) acids.